regulation of bone development [GO:1903010] (biological process) Subtypes: GO:1902738, negative regulation of bone development [GO:1903011], GO:1903012 References: PMID:22510437 Sources: GOC:TermGenie, GOC:mr, GO_REF:0000058 Relationships: is a type of regulation of multicellular organismal development [GO:2000026]; regulates bone development [GO:0060348] Definition: Any process that modulates the frequency, rate or extent of bone development.